{
  "gene": "UniProtKB:Q9Y5G4",
  "term_id": "GO:0005886",
  "gene_name": "Protocadherin gamma-A9",
  "gene_symbol": "PCDHGA9",
  "term_label": "plasma membrane"
}